AnxA2-p11 complex [GO:1990665] (cellular component) Relationships: is a type of protein-containing complex [GO:0032991] References: PMID:18799458, PMID:23483454 Sources: GOC:BHF, GOC:bf, GOC:nc Also known as: (A2.p11)2 complex, (p11)2.(AnxA2)2 complex, Annexin A2-p11 complex, AnxA2.p11 complex, AnxA2:S100A10 heterotetramer, Annexin A2 tetramer Definition: A heterotetrameric protein complex comprising two Annexin A2 (AnxA2) monomers and two copies of its binding partner, S100 protein p11 (S100A10).